{
  "term_label": "nucleus",
  "gene_symbol": "RFXANK",
  "gene_name": "DNA-binding protein RFXANK",
  "gene": "UniProtKB:O14593",
  "term_id": "GO:0005634"
}